{
  "term_id": "GO:0007265",
  "gene_name": "Ras suppressor protein 1",
  "term_label": "Ras protein signal transduction",
  "gene_symbol": "RSU1",
  "gene": "UniProtKB:Q15404"
}